{
  "term_label": "glucokinase activity",
  "gene_name": "Hexokinase-3",
  "gene_symbol": "HK3",
  "term_id": "GO:0004340",
  "gene": "UniProtKB:P52790"
}